{
  "term_id": "UNKNOWN:0002",
  "gene": "UniProtKB:Q5VYM1",
  "term_label": "Unknown biological process",
  "gene_name": "Uncharacterized protein C9orf131",
  "gene_symbol": "C9orf131"
}